{
  "term_label": "serine-type endopeptidase activity",
  "gene_name": "Tryptase beta-2",
  "gene": "UniProtKB:P20231",
  "gene_symbol": "TPSB2",
  "term_id": "GO:0004252"
}